{
  "term_id": "GO:0008285",
  "gene_symbol": "SAV1",
  "gene_name": "Protein salvador homolog 1",
  "term_label": "negative regulation of cell population proliferation",
  "gene": "UniProtKB:Q9H4B6"
}